{
  "term_label": "endoplasmic reticulum-plasma membrane contact site",
  "gene": "UniProtKB:Q3KR37",
  "term_id": "GO:0140268",
  "gene_symbol": "GRAMD1B",
  "gene_name": "Protein Aster-B"
}